{
  "gene_name": "Myocardin-related transcription factor A",
  "gene_symbol": "MRTFA",
  "term_id": "GO:0045944",
  "term_label": "positive regulation of transcription by RNA polymerase II",
  "gene": "UniProtKB:Q969V6"
}